{
  "term_id": "GO:0002227",
  "gene": "UniProtKB:Q6DN03",
  "term_label": "innate immune response in mucosa",
  "gene_name": "Putative histone H2B type 2-C",
  "gene_symbol": "H2BC20P"
}